regulation of epithelial cell apoptotic process [GO:1904035] (biological process) Relationships: is a type of regulation of apoptotic process [GO:0042981]; regulates epithelial cell apoptotic process [GO:1904019] References: PMID:19137015 Sources: GOC:TermGenie, GO_REF:0000058 Also known as: regulation of epitheliocyte apoptotic process, regulation of epithelial cell apoptosis, regulation of epitheliocyte apoptosis Subtypes: regulation of keratinocyte apoptotic process [GO:1902172], regulation of hepatocyte apoptotic process [GO:1903943], negative regulation of epithelial cell apoptotic process [GO:1904036], positive regulation of epithelial cell apoptotic process [GO:1904037], regulation of cholangiocyte apoptotic process [GO:1904192], GO:1904633, regulation of granulosa cell apoptotic process [GO:1904708], regulation of type B pancreatic cell apoptotic process [GO:2000674] Definition: Any process that modulates the frequency, rate or extent of epithelial cell apoptotic process.